{
  "gene": "UniProtKB:A0A0K0K1A3",
  "term_id": "UNKNOWN:0001",
  "gene_name": "T cell receptor beta variable 10-1",
  "term_label": "Unknown molecular function",
  "gene_symbol": "TRBV10-1"
}